{
  "gene": "UniProtKB:Q8IYL9",
  "term_id": "GO:0007189",
  "gene_symbol": "GPR65",
  "term_label": "adenylate cyclase-activating G protein-coupled receptor signaling pathway",
  "gene_name": "Psychosine receptor"
}